{
  "gene": "UniProtKB:Q96QS6",
  "gene_name": "Serine_threonine-protein kinase H2",
  "term_id": "UNKNOWN:0002",
  "gene_symbol": "PSKH2",
  "term_label": "Unknown biological process"
}